{
  "term_label": "positive regulation of heart rate",
  "gene_symbol": "ADM5",
  "gene_name": "Putative adrenomedullin-5-like protein",
  "gene": "UniProtKB:C9JUS6",
  "term_id": "GO:0010460"
}